GTP cyclohydrolase I regulator activity [GO:0060308] (molecular function) Relationships: is a type of enzyme regulator activity [GO:0030234]; has part GTP cyclohydrolase binding [GO:0044549]; regulates GTP cyclohydrolase I activity [GO:0003934] Definition: Binds to and modulates the activity of GTP cyclohydrolase I. GTP cyclohydrolase I activity catalyzes the reaction: GTP + 2 H2O = formate + 2-amino-4-hydroxy-6-(erythro-1,2,3-trihydroxypropyl)-dihydropteridine triphosphate. Sources: GOC:dph, GOC:tb